{
  "gene_name": "COP9 signalosome complex subunit 7a",
  "gene_symbol": "COPS7A",
  "gene": "UniProtKB:Q9UBW8",
  "term_id": "GO:0008180",
  "term_label": "COP9 signalosome"
}